{
  "term_label": "regulation of microtubule polymerization or depolymerization",
  "gene_name": "Spindle and kinetochore-associated protein 1",
  "gene_symbol": "SKA1",
  "term_id": "GO:0031110",
  "gene": "UniProtKB:Q96BD8"
}